dendrite regeneration [GO:0031104] (biological process) Relationships: is a type of dendrite development [GO:0016358]; is a type of neuron projection regeneration [GO:0031102] Definition: The regrowth of dendrites in response to their loss or damage. Sources: GOC:dgh, GOC:dph, GOC:tb